{
  "term_label": "water transport",
  "gene_symbol": "AQP4",
  "term_id": "GO:0006833",
  "gene_name": "Aquaporin-4",
  "gene": "UniProtKB:P55087"
}